{
  "gene_name": "Microtubule-associated serine_threonine-protein kinase 2",
  "term_id": "GO:0015630",
  "gene_symbol": "MAST2",
  "gene": "UniProtKB:Q6P0Q8",
  "term_label": "microtubule cytoskeleton"
}